{
  "gene": "UniProtKB:Q9H8S9",
  "term_label": "protein kinase activator activity",
  "gene_symbol": "MOB1A",
  "gene_name": "MOB kinase activator 1A",
  "term_id": "GO:0030295"
}